{
  "term_label": "nucleus",
  "gene": "UniProtKB:Q01844",
  "term_id": "GO:0005634",
  "gene_name": "RNA-binding protein EWS",
  "gene_symbol": "EWSR1"
}